{
  "gene": "UniProtKB:Q92539",
  "term_label": "phosphatidate phosphatase activity",
  "term_id": "GO:0008195",
  "gene_name": "Phosphatidate phosphatase LPIN2",
  "gene_symbol": "LPIN2"
}